dorsal trunk growth, open tracheal system [GO:0035001] (BP) Definition: Growth of epithelial tubes that originate from pits in an open tracheal system and grow towards each other to meet and form a continuous open tube called the dorsal trunk. The dorsal trunk extends from the anterior spiracle to the posterior spiracle of the larva and forms the main airway of the insect tracheal system. Sources: GOC:mtg_sensu, ISBN:0879694238 Also known as: dorsal trunk growth Relationships: is a type of developmental growth involved in morphogenesis [GO:0060560]; is part of GO:0007424